activation of GTPase activity [GO:0090630] (BP) Also known as: ARF GTPase activation, Cdc42 GTPase activation, Rab GTPase activation, Rac GTPase activation, Ral GTPase activation, Ran GTPase activation, Rap GTPase activation, Ras GTPase activation, Rho GTPase activation, activation of ARF GTPase activity, activation of Cdc42 GTPase activity, activation of Rab GTPase activity, activation of Rac GTPase activity, activation of Ral GTPase activity, activation of Ran GTPase activity, activation of Rap GTPase activity, activation of Ras GTPase activity, activation of Rho GTPase activity Relationships: is a type of GO:0043547 Definition: Any process that initiates the activity of an inactive GTPase through the replacement of GDP by GTP. Sources: GOC:dph, GOC:mah, GOC:tb